{
  "term_label": "transcription corepressor activity",
  "gene_name": "Protein Tob2",
  "term_id": "GO:0003714",
  "gene": "UniProtKB:Q14106",
  "gene_symbol": "TOB2"
}